{
  "gene_symbol": "MANBAL",
  "gene": "UniProtKB:Q9NQG1",
  "term_id": "UNKNOWN:0003",
  "term_label": "Unknown cellular component",
  "gene_name": "Protein MANBAL"
}